protein depalmitoleylation [GO:1990697] (biological process) Relationships: is a type of GO:0035601; is a type of lipoprotein catabolic process [GO:0042159] Definition: The removal of palmitoleyl group, a 16-carbon monounsaturated fatty acid (C16:1), from a lipoprotein. References: PMID:25731175